phosphatidic acid metabolic process [GO:0046473] (biological process) Definition: The chemical reactions and pathways involving phosphatidic acid, any derivative of glycerol phosphate in which both the remaining hydroxyl groups of the glycerol moiety are esterified with fatty acids. Relationships: is a type of glycerophospholipid metabolic process [GO:0006650] Subtypes: phosphatidic acid biosynthetic process [GO:0006654] Sources: ISBN:0198506732 Also known as: phosphatidic acid metabolism